{
  "term_label": "tRNA pseudouridine synthesis",
  "term_id": "GO:0031119",
  "gene": "UniProtKB:Q3MIT2",
  "gene_name": "tRNA pseudouridine synthase Pus10",
  "gene_symbol": "PUS10"
}